{
  "gene": "UniProtKB:Q9HB29",
  "term_label": "Unknown molecular function",
  "gene_symbol": "IL1RL2",
  "term_id": "UNKNOWN:0001",
  "gene_name": "Interleukin-1 receptor-like 2"
}